{
  "term_id": "GO:0046928",
  "gene": "UniProtKB:Q9HC10",
  "gene_name": "Otoferlin",
  "term_label": "regulation of neurotransmitter secretion",
  "gene_symbol": "OTOF"
}